{
  "term_id": "UNKNOWN:0001",
  "gene_name": "T cell receptor delta variable 2",
  "gene_symbol": "TRDV2",
  "gene": "UniProtKB:A0JD36",
  "term_label": "Unknown molecular function"
}